phthalate catabolic process [GO:0046239] (biological process) Relationships: is a type of phthalate metabolic process [GO:0018963]; is a type of xenobiotic catabolic process [GO:0042178]; is a type of carboxylic acid catabolic process [GO:0046395] Definition: The chemical reactions and pathways resulting in the breakdown of phthalate, the anion of phthalic acid. Sources: GOC:ai Also known as: phthalate breakdown, phthalate catabolism, phthalate degradation